{
  "term_id": "UNKNOWN:0002",
  "term_label": "Unknown biological process",
  "gene": "UniProtKB:Q86TH1",
  "gene_symbol": "ADAMTSL2",
  "gene_name": "ADAMTS-like protein 2"
}